regulation of gonad development [GO:1905939] (biological process) Definition: Any process that modulates the frequency, rate or extent of gonad development. References: PMID:15342467 Sources: GOC:TermGenie, GO_REF:0000058 Also known as: regulation of gonadogenesis Relationships: is a type of regulation of developmental process [GO:0050793]; is a type of regulation of reproductive process [GO:2000241]; regulates gonad development [GO:0008406] Subtypes: negative regulation of gonad development [GO:1905940], positive regulation of gonad development [GO:1905941], GO:2000018, GO:2000194